{
  "gene_symbol": "OR2A1",
  "term_id": "UNKNOWN:0003",
  "gene_name": "Olfactory receptor",
  "term_label": "Unknown cellular component",
  "gene": "UniProtKB:A0A2R8YEG4"
}